{
  "gene_name": "Zinc finger protein 69",
  "gene": "UniProtKB:Q9UC07",
  "term_id": "GO:0000977",
  "gene_symbol": "ZNF69",
  "term_label": "RNA polymerase II transcription regulatory region sequence-specific DNA binding"
}